{
  "gene_name": "Aldo-keto reductase family 1 member C1",
  "gene_symbol": "AKR1C1",
  "term_id": "GO:0042448",
  "gene": "UniProtKB:Q04828",
  "term_label": "progesterone metabolic process"
}